{
  "term_id": "GO:0003333",
  "term_label": "amino acid transmembrane transport",
  "gene_name": "Sodium-coupled neutral amino acid symporter 1",
  "gene": "UniProtKB:Q9H2H9",
  "gene_symbol": "SLC38A1"
}